{
  "gene": "UniProtKB:P0CG01",
  "term_id": "GO:0042127",
  "gene_name": "Gastrokine-3",
  "term_label": "regulation of cell population proliferation",
  "gene_symbol": "GKN3P"
}